{
  "gene_name": "Adenylate cyclase type 4",
  "term_label": "cAMP biosynthetic process",
  "term_id": "GO:0006171",
  "gene": "UniProtKB:Q8NFM4",
  "gene_symbol": "ADCY4"
}